{
  "term_id": "GO:0000978",
  "term_label": "RNA polymerase II cis-regulatory region sequence-specific DNA binding",
  "gene_name": "Retina and anterior neural fold homeobox protein 2",
  "gene_symbol": "RAX2",
  "gene": "UniProtKB:Q96IS3"
}